transcription by RNA polymerase II [GO:0006366] (biological process) Subtypes: snoRNA transcription by RNA polymerase II [GO:0001015], GO:0042789, snRNA transcription by RNA polymerase II [GO:0042795] Relationships: is_a DNA-templated transcription [GO:0006351] Also known as: transcription from Pol II promoter, transcription from RNA polymerase II promoter, RNA polymerase II transcription factor activity, gene-specific transcription from RNA polymerase II promoter, general transcription from RNA polymerase II promoter, specific transcription from RNA polymerase II promoter Definition: The synthesis of RNA from a DNA template by RNA polymerase II (RNAP II), originating at an RNA polymerase II promoter. Includes transcription of messenger RNA (mRNA) and certain small nuclear RNAs (snRNAs). Regulation: negatively regulated by GO:0000122; regulated by regulation of transcription by RNA polymerase II [GO:0006357]; RO_0002213 by positive regulation of transcription by RNA polymerase II [GO:0045944] Sources: GOC:jl, GOC:txnOH, ISBN:0321000382